{
  "term_label": "Unknown cellular component",
  "gene_symbol": "VCX3B",
  "gene_name": "Variable charge X-linked protein 3B",
  "gene": "UniProtKB:Q9H321",
  "term_id": "UNKNOWN:0003"
}